{
  "gene_name": "Hexokinase-3",
  "gene": "UniProtKB:P52790",
  "term_label": "glucose 6-phosphate metabolic process",
  "term_id": "GO:0051156",
  "gene_symbol": "HK3"
}